regulation of vacuolar transport [GO:1903335] (biological process) Sources: GOC:TermGenie, GOC:vw, GO_REF:0000058 Definition: Any process that modulates the frequency, rate or extent of vacuolar transport. Subtypes: regulation of protein targeting to vacuolar membrane [GO:1900483], regulation of late endosome to lysosome transport [GO:1902822], negative regulation of vacuolar transport [GO:1903336], positive regulation of vacuolar transport [GO:1903337], GO:1904051, regulation of protein localization by the Cvt pathway [GO:2001159] Relationships: is a type of regulation of intracellular transport [GO:0032386]; regulates GO:0007034